{
  "gene": "UniProtKB:Q6NXT2",
  "gene_name": "Histone H3.3C",
  "term_label": "structural constituent of chromatin",
  "term_id": "GO:0030527",
  "gene_symbol": "H3-5"
}